{
  "gene_name": "Sorbin and SH3 domain-containing protein 2",
  "gene": "UniProtKB:O94875",
  "term_id": "GO:0005886",
  "gene_symbol": "SORBS2",
  "term_label": "plasma membrane"
}